{
  "term_id": "GO:1990756",
  "gene": "UniProtKB:Q53GT1",
  "gene_name": "Kelch-like protein 22",
  "gene_symbol": "KLHL22",
  "term_label": "ubiquitin-like ligase-substrate adaptor activity"
}